glyceollin synthase activity [GO:0033769] (molecular function) Definition: Catalysis of the reactions: 2-dimethylallyl-(6aS,11aS)-3,6a,9-trihydroxypterocarpan + NADPH + H+ + O2 = glyceollin II or glyceollin III + NADP+ + 2 H2O, and 4-dimethylallyl-(6aS,11aS)-3,6a,9-trihydroxypterocarpan + NADPH + H+ + O2 = glyceollin I + NADP+ + 2 H2O. Also known as: dimethylallyl-3,6a,9-trihydroxypterocarpan cyclase activity Sources: EC:1.14.14.135 Relationships: is_a oxidoreductase activity, acting on paired donors, with incorporation or reduction of molecular oxygen, reduced flavin or flavoprotein as one donor, and incorporation of one atom of oxygen [GO:0016712]